{
  "gene": "UniProtKB:P04075",
  "term_id": "GO:0005829",
  "gene_symbol": "ALDOA",
  "gene_name": "Fructose-bisphosphate aldolase A",
  "term_label": "cytosol"
}